{
  "gene_name": "REST corepressor 2",
  "gene_symbol": "RCOR2",
  "term_label": "negative regulation of DNA-templated transcription",
  "gene": "UniProtKB:Q8IZ40",
  "term_id": "GO:0045892"
}